{
  "gene_name": "Uncharacterized protein",
  "gene_symbol": "A0A6Q8PGL7",
  "term_label": "Unknown cellular component",
  "term_id": "UNKNOWN:0003",
  "gene": "UniProtKB:A0A6Q8PGL7"
}